{
  "term_id": "UNKNOWN:0001",
  "gene": "UniProtKB:A0A087WTH1",
  "gene_symbol": "TMEM265",
  "term_label": "Unknown molecular function",
  "gene_name": "Transmembrane protein 265"
}